B-1 B cell differentiation [GO:0001923] (biological process) Relationships: is a type of mature B cell differentiation [GO:0002335] Definition: The process in which a hemopoietic stem cell acquires the specialized features of a B-1 B cell. B-1 B cells are a distinct subset of B cells characterized as being CD5 positive, found predominantly in the peritoneum, pleural cavities, and spleen, and enriched for self-reactivity. Sources: GOC:add, ISBN:0781735149 Regulation: regulated by regulation of B-1 B cell differentiation [GO:0001924]; negatively regulated by negative regulation of B-1 B cell differentiation [GO:0001925]; positively regulated by positive regulation of B-1 B cell differentiation [GO:0001926] Also known as: B-1 B lymphocyte differentiation, B-1 B-cell differentiation, B-1 B-lymphocyte differentiation, B-1 B cell development Subtypes: GO:0002337, GO:0002338